{
  "term_label": "integrin-mediated signaling pathway",
  "gene_symbol": "ITGAV",
  "gene": "UniProtKB:P06756",
  "gene_name": "Integrin alpha-V",
  "term_id": "GO:0007229"
}